{
  "gene_name": "Tyrosine-protein kinase HCK",
  "gene_symbol": "HCK",
  "term_label": "cell surface receptor protein tyrosine kinase signaling pathway",
  "term_id": "GO:0007169",
  "gene": "UniProtKB:P08631"
}